L-tyrosine catabolic process [GO:0006572] (biological process) Sources: GOC:go_curators Subtypes: L-tyrosine catabolic process to fumarate [GO:0019445] Definition: The chemical reactions and pathways resulting in the breakdown of L-tyrosine, an aromatic amino acid, 2-amino-3-(4-hydroxyphenyl)propanoic acid. Relationships: is a type of tyrosine metabolic process [GO:0006570]; is a type of aromatic amino acid family catabolic process [GO:0009074]; is a type of L-amino acid catabolic process [GO:0170035]; is a type of proteinogenic amino acid catabolic process [GO:0170040] Also known as: tyrosine breakdown, tyrosine catabolism, tyrosine degradation